{
  "gene_name": "Eukaryotic translation initiation factor 2D",
  "term_label": "translation initiation factor activity",
  "gene": "UniProtKB:P41214",
  "gene_symbol": "EIF2D",
  "term_id": "GO:0003743"
}